{
  "gene_symbol": "IGHV3-16",
  "term_label": "Unknown cellular component",
  "gene": "UniProtKB:A0A0C4DH30",
  "term_id": "UNKNOWN:0003",
  "gene_name": "Probable non-functional immunoglobulin heavy variable 3-16"
}